{
  "gene_symbol": "PINK1",
  "gene": "UniProtKB:Q9BXM7",
  "term_id": "GO:0042981",
  "gene_name": "Serine_threonine-protein kinase PINK1, mitochondrial",
  "term_label": "regulation of apoptotic process"
}